proline 3-hydroxylase activity [GO:0033763] (molecular function) Definition: Catalysis of the reaction: L-proline + 2-oxoglutarate + O2 = cis-3-hydroxy-L-proline + succinate + CO2. Sources: EC:1.14.11.28 Also known as: L-proline,2-oxoglutarate:oxygen oxidoreductase (3-hydroxylating) activity, P-3-H Relationships: is a type of 2-oxoglutarate-dependent dioxygenase activity [GO:0016706]